{
  "gene_symbol": "CTF1",
  "term_id": "GO:0005576",
  "gene_name": "Cardiotrophin-1",
  "gene": "UniProtKB:Q16619",
  "term_label": "extracellular region"
}